{
  "term_id": "UNKNOWN:0002",
  "term_label": "Unknown biological process",
  "gene": "UniProtKB:P62502",
  "gene_symbol": "LCN6",
  "gene_name": "Epididymal-specific lipocalin-6"
}